{
  "gene_name": "Reticulocalbin-2",
  "term_label": "endoplasmic reticulum",
  "gene_symbol": "RCN2",
  "term_id": "GO:0005783",
  "gene": "UniProtKB:Q14257"
}